{
  "gene_symbol": "UIMC1",
  "term_id": "GO:0070530",
  "gene": "UniProtKB:Q96RL1",
  "gene_name": "BRCA1-A complex subunit RAP80",
  "term_label": "K63-linked polyubiquitin modification-dependent protein binding"
}